{
  "term_id": "GO:0034246",
  "gene_symbol": "TFB2M",
  "gene_name": "Dimethyladenosine transferase 2, mitochondrial",
  "gene": "UniProtKB:Q9H5Q4",
  "term_label": "mitochondrial transcription factor activity"
}